{
  "term_id": "GO:0005643",
  "gene": "UniProtKB:Q12769",
  "gene_name": "Nuclear pore complex protein Nup160",
  "gene_symbol": "NUP160",
  "term_label": "nuclear pore"
}